{
  "gene_symbol": "PDLIM3",
  "gene_name": "PDZ and LIM domain protein 3",
  "term_id": "GO:0051371",
  "gene": "UniProtKB:Q53GG5",
  "term_label": "muscle alpha-actinin binding"
}